{
  "term_id": "GO:0008239",
  "gene_symbol": "DPP9",
  "gene_name": "Dipeptidyl peptidase 9",
  "gene": "UniProtKB:Q86TI2",
  "term_label": "dipeptidyl-peptidase activity"
}